{
  "term_label": "transcription coactivator activity",
  "gene_name": "Transcriptional coactivator YAP1",
  "term_id": "GO:0003713",
  "gene_symbol": "YAP1",
  "gene": "UniProtKB:P46937"
}